{
  "gene_symbol": "TMPRSS12",
  "term_label": "acrosomal vesicle",
  "gene_name": "Transmembrane protease serine 12",
  "term_id": "GO:0001669",
  "gene": "UniProtKB:Q86WS5"
}